mannose transmembrane transporter activity [GO:0015578] (molecular function) Also known as: mannose permease activity Subtypes: GO:0022870, mannose:proton symporter activity [GO:0055053], GO:0140929 Relationships: is a type of GO:0015149; is part of GO:0015761 Sources: GOC:ai, GOC:mtg_transport, ISBN:0815340729 Definition: Enables the transfer of mannose from one side of a membrane to the other. Mannose is the aldohexose manno-hexose, the C-2 epimer of glucose. The D-(+)-form is widely distributed in mannans and hemicelluloses and is of major importance in the core oligosaccharide of N-linked oligosaccharides of glycoproteins.